lactose catabolic process via UDP-galactose [GO:0019515] (biological process) Definition: The chemical reactions and pathways resulting in the breakdown of lactose, via the intermediate UDP-galactose. Sources: GOC:go_curators Also known as: lactose breakdown via UDP-galactose, lactose degradation via UDP-galactose Relationships: is a type of GO:0005990